{
  "gene_name": "Putative olfactory receptor 3A4",
  "gene": "UniProtKB:P47883",
  "gene_symbol": "OR3A4P",
  "term_label": "signal transduction",
  "term_id": "GO:0007165"
}